{
  "gene_name": "Phosphatidylinositol 4-phosphate 3-kinase C2 domain-containing subunit alpha",
  "term_id": "GO:0016477",
  "gene_symbol": "PIK3C2A",
  "gene": "UniProtKB:O00443",
  "term_label": "cell migration"
}